{
  "gene_name": "ADP-ribosylhydrolase ARH3",
  "term_label": "peptidyl-serine ADP-deribosylation",
  "term_id": "GO:0140290",
  "gene": "UniProtKB:Q9NX46",
  "gene_symbol": "ADPRS"
}